{
  "gene_name": "Serine_threonine-protein kinase PRP4 homolog",
  "term_id": "GO:0004674",
  "term_label": "protein serine/threonine kinase activity",
  "gene": "UniProtKB:Q13523",
  "gene_symbol": "PRPF4B"
}